{
  "term_label": "epithelial cell differentiation",
  "gene_name": "Keratin, type I cuticular Ha5",
  "term_id": "GO:0030855",
  "gene": "UniProtKB:Q92764",
  "gene_symbol": "KRT35"
}